uridine phosphorylase activity [GO:0004850] (molecular function) Definition: Catalysis of the reaction: uridine + phosphate = uracil + alpha-D-ribose 1-phosphate. Sources: EC:2.4.2.3 Also known as: pyrimidine phosphorylase activity, UPH, UPase activity, UrdPase activity, uridine:phosphate alpha-D-ribosyltransferase activity Relationships: is a type of pyrimidine-nucleoside phosphorylase activity [GO:0016154]